{
  "term_label": "nucleosome assembly",
  "gene": "UniProtKB:Q99733",
  "term_id": "GO:0006334",
  "gene_name": "Nucleosome assembly protein 1-like 4",
  "gene_symbol": "NAP1L4"
}